{
  "term_label": "axoneme",
  "gene_name": "Intraflagellar transport protein 140 homolog",
  "gene": "UniProtKB:Q96RY7",
  "term_id": "GO:0005930",
  "gene_symbol": "IFT140"
}